{
  "term_id": "GO:0045087",
  "gene_name": "Ankyrin repeat and KH domain-containing protein 1",
  "gene_symbol": "ANKHD1",
  "gene": "UniProtKB:Q8IWZ3",
  "term_label": "innate immune response"
}